regulation of asperthecin biosynthetic process [GO:1900379] (biological process) Definition: Any process that modulates the frequency, rate or extent of asperthecin biosynthetic process. Subtypes: negative regulation of asperthecin biosynthetic process [GO:1900380], positive regulation of asperthecin biosynthetic process [GO:1900381] Relationships: is a type of regulation of ketone biosynthetic process [GO:0010566]; is a type of regulation of secondary metabolite biosynthetic process [GO:1900376]; regulates asperthecin biosynthetic process [GO:0036184] Sources: GOC:TermGenie, GOC:di Also known as: regulation of asperthecin biosynthesis, regulation of asperthecin formation, regulation of asperthecin synthesis